{
  "gene": "UniProtKB:Q8TD57",
  "gene_name": "Dynein axonemal heavy chain 3",
  "term_label": "cilium movement involved in cell motility",
  "term_id": "GO:0060294",
  "gene_symbol": "DNAH3"
}